{
  "gene_name": "Putative WAS protein family homolog 4",
  "gene_symbol": "WASH4P",
  "term_id": "GO:0034314",
  "term_label": "Arp2/3 complex-mediated actin nucleation",
  "gene": "UniProtKB:A8MWX3"
}